{
  "gene_name": "PPP2R1A-PPP2R2A-interacting phosphatase regulator 1",
  "term_label": "positive regulation of proteasomal ubiquitin-dependent protein catabolic process",
  "gene": "UniProtKB:Q96E09",
  "gene_symbol": "PABIR1",
  "term_id": "GO:0032436"
}